{
  "gene_name": "Putative inactive carbonic anhydrase 5B-like protein",
  "term_id": "GO:0005737",
  "term_label": "cytoplasm",
  "gene_symbol": "CA5BP1",
  "gene": "UniProtKB:Q8WTZ4"
}